negative regulation of aldosterone biosynthetic process [GO:0032348] (biological process) Sources: GOC:mah Also known as: down regulation of aldosterone biosynthetic process, down-regulation of aldosterone biosynthetic process, downregulation of aldosterone biosynthetic process, inhibition of aldosterone biosynthetic process Relationships: is a type of regulation of aldosterone biosynthetic process [GO:0032347]; is a type of negative regulation of steroid hormone biosynthetic process [GO:0090032]; is a type of GO:1902931; negatively regulates aldosterone biosynthetic process [GO:0032342] Definition: Any process that stops, prevents, or reduces the frequency, rate or extent of the chemical reactions and pathways resulting in the formation of aldosterone.